{
  "term_label": "Unknown molecular function",
  "term_id": "UNKNOWN:0001",
  "gene_symbol": "CEP44",
  "gene_name": "Centrosomal protein of 44 kDa",
  "gene": "UniProtKB:Q9C0F1"
}